symbiont-mediated disruption of host cellular anatomical structure [GO:0052008] (biological process) Definition: The process in which an organism effects a change that impairs the structure or function of a host cellular anatomical structure. The host is defined as the larger of the organisms involved in a symbiotic interaction. Also known as: symbiont-mediated disruption of host cellular component, catabolism of host cellular component by organism, catabolism of host structural constituent by organism, degradation of host cellular component by organism, disassembly by organism of host cellular component, disruption by symbiont of host cellular component, symbiont-mediated disruption of host cellular anatomical entity, cytopathogenic effect, disassembly by symbiont of host cellular component Sources: ISBN:0198547684 Relationships: is a type of GO:0052111 Subtypes: symbiont-mediated disruption of host chloroplast [GO:0033656], symbiont-mediated disruption of host chloroplast thylakoid [GO:0033658], symbiont-mediated disruption of host mitochondrion [GO:0033659], symbiont-mediated disruption of host cell nucleus [GO:0044066], symbiont-mediated perturbation of host cell-cell junction [GO:0044067], symbiont-mediated perturbation of host cytoskeleton [GO:0052039], symbiont-mediated disruption of host cell PML body [GO:0075342], GO:0098933, symbiont-mediated disruption of host focal adhesion [GO:0141029], GO:0141066, symbiont-mediated disruption of host neutrophil extracellular traps [GO:0141144], symbiont-mediated disruption of host phagosome [GO:0141160], GO:0141171